pentadecane metabolic process [GO:1900633] (BP) Subtypes: GO:1900634 Relationships: is a type of hydrocarbon metabolic process [GO:0120252] Also known as: pentadecane metabolism Sources: GOC:TermGenie, GOC:mengo_curators Definition: The chemical reactions and pathways involving pentadecane.